{
  "gene_name": "Importin-5",
  "term_label": "nucleus",
  "gene_symbol": "IPO5",
  "gene": "UniProtKB:O00410",
  "term_id": "GO:0005634"
}